{
  "gene": "UniProtKB:Q9C035",
  "gene_name": "Tripartite motif-containing protein 5",
  "term_id": "GO:0010468",
  "term_label": "regulation of gene expression",
  "gene_symbol": "TRIM5"
}